{
  "gene_name": "Putative neuroblastoma breakpoint family member 7",
  "gene": "UniProtKB:P0C2Y1",
  "term_id": "UNKNOWN:0001",
  "term_label": "Unknown molecular function",
  "gene_symbol": "NBPF7P"
}